ammonia oxidation [GO:0019329] (biological process) Definition: The chemical reactions and pathways by which ammonia or ammonium is converted to molecular nitrogen or another nitrogen compound, with accompanying loss of electrons. Relationships: is a type of small molecule metabolic process [GO:0044281] Sources: GOC:mah Subtypes: anaerobic respiration, using ammonium as electron donor [GO:0019331], aerobic respiration, using ammonia as electron donor [GO:0019409], aerobic ammonia oxidation to nitrite via pyruvic oxime [GO:0070275]